{
  "gene_name": "E3 ubiquitin-protein ligase CBL",
  "term_label": "negative regulation of epidermal growth factor receptor signaling pathway",
  "gene_symbol": "CBL",
  "term_id": "GO:0042059",
  "gene": "UniProtKB:P22681"
}